{
  "gene_symbol": "ARHGEF9",
  "term_id": "GO:0098982",
  "gene_name": "Rho guanine nucleotide exchange factor 9",
  "gene": "UniProtKB:O43307",
  "term_label": "GABA-ergic synapse"
}